cellular response to jasmonic acid stimulus [GO:0071395] (BP) Definition: Any process that results in a change in state or activity of a cell (in terms of movement, secretion, enzyme production, gene expression, etc.) as a result of a jasmonic acid stimulus. Sources: GOC:mah Relationships: is a type of response to jasmonic acid [GO:0009753]; is a type of cellular response to hormone stimulus [GO:0032870]; is a type of cellular response to fatty acid [GO:0071398]